{
  "gene": "UniProtKB:Q9NYL5",
  "term_id": "GO:0006699",
  "term_label": "bile acid biosynthetic process",
  "gene_symbol": "CYP39A1",
  "gene_name": "24-hydroxycholesterol 7-alpha-hydroxylase"
}